{
  "term_id": "GO:0005764",
  "term_label": "lysosome",
  "gene_name": "Beta-hexosaminidase subunit beta",
  "gene": "UniProtKB:P07686",
  "gene_symbol": "HEXB"
}